negative regulation of spore-bearing organ development [GO:0075262] (biological process) Definition: Any process that stops, prevents, or reduces the frequency, rate or extent of spore-bearing organ development, a process in which hyphae grow into special aggregates called fruiting bodies that produce new spores. Sources: GOC:pamgo_curators Relationships: is_a negative regulation of developmental process [GO:0051093]; is a type of GO:0051241; is a type of GO:0075260; is a type of negative regulation of reproductive process [GO:2000242]; negatively regulates GO:0075259 Subtypes: negative regulation of sorocarp stalk cell differentiation [GO:0031286], negative regulation of conidiophore development [GO:0070794], negative regulation of oogonium development [GO:0075266], GO:0075270, negative regulation of zygosporangium development [GO:0075274], negative regulation of telium development [GO:0075278], negative regulation of uredinium development [GO:0075282], negative regulation of sporangium development [GO:0075312], negative regulation of basidium development [GO:0075316], negative regulation of ascus development [GO:0075320], negative regulation of sporocarp development involved in sexual reproduction [GO:1902059]